{
  "gene_symbol": "KIF18A",
  "term_label": "mitotic sister chromatid segregation",
  "gene_name": "Kinesin-like protein KIF18A",
  "term_id": "GO:0000070",
  "gene": "UniProtKB:Q8NI77"
}